{
  "gene_symbol": "EPHB6",
  "gene": "UniProtKB:O15197",
  "term_id": "GO:0007411",
  "gene_name": "Ephrin type-B receptor 6",
  "term_label": "axon guidance"
}